{
  "term_id": "UNKNOWN:0003",
  "gene_name": "Protein BNIP5",
  "gene": "UniProtKB:P0C671",
  "gene_symbol": "BNIP5",
  "term_label": "Unknown cellular component"
}